positive regulation of telomere maintenance via telomerase [GO:0032212] (biological process) Also known as: up regulation of telomere maintenance via telomerase activity, up-regulation of telomere maintenance via telomerase activity, upregulation of telomere maintenance via telomerase activity, activation of telomere maintenance via telomerase, stimulation of telomere maintenance via telomerase Sources: GOC:mah Definition: Any process that activates or increases the frequency, rate or extent of the addition of telomeric repeats by telomerase. Relationships: is a type of regulation of telomere maintenance via telomerase [GO:0032210]; is a type of GO:1904358; is a type of positive regulation of DNA biosynthetic process [GO:2000573]; positively regulates telomere maintenance via telomerase [GO:0007004]